{
  "gene": "UniProtKB:Q9BQ83",
  "gene_symbol": "SLX1A",
  "gene_name": "Structure-specific endonuclease subunit SLX1",
  "term_label": "Slx1-Slx4 complex",
  "term_id": "GO:0033557"
}